methyl tert-butyl ether metabolic process [GO:0018906] (biological process) Definition: The chemical reactions and pathways involving methyl tert-butyl ether, 2-methoxy-2-methylpropane. Methyl tert-butyl ether is a synthetic chemical which is mixed with gasoline for use in reformulated gasoline. It was first introduced as an additive for unleaded gasoline in the 1980s. It is also used as a laboratory reagent and a pharmaceutical agent. Relationships: is_a GO:0006805 Also known as: methyl tert-butyl ether metabolism Sources: UM-BBD_pathwayID:mtb